{
  "term_id": "UNKNOWN:0001",
  "gene_symbol": "ZDBF2",
  "gene": "UniProtKB:Q9HCK1",
  "gene_name": "DBF4-type zinc finger-containing protein 2",
  "term_label": "Unknown molecular function"
}